{
  "term_label": "dendrite",
  "term_id": "GO:0030425",
  "gene_symbol": "CNIH2",
  "gene": "UniProtKB:Q6PI25",
  "gene_name": "Protein cornichon homolog 2"
}